{
  "gene_symbol": "DNAI2",
  "term_label": "cilium movement",
  "gene_name": "Dynein axonemal intermediate chain 2",
  "gene": "UniProtKB:Q9GZS0",
  "term_id": "GO:0003341"
}